negative regulation of cristae formation [GO:1903851] (biological process) Also known as: down regulation of cristae formation, down-regulation of cristae formation, downregulation of cristae formation, inhibition of cristae formation References: PMID:19279012 Sources: GOC:PARL, GOC:TermGenie, GOC:pad, GO_REF:0000058 Note: AN example of this is PINK1 in human (Q9BXM7) in PMID:19279012 inferred from mutant phenotype Relationships: is a type of negative regulation of organelle organization [GO:0010639]; is a type of regulation of cristae formation [GO:1903850]; negatively regulates cristae formation [GO:0042407] Definition: Any process that stops, prevents or reduces the frequency, rate or extent of cristae formation.